{
  "term_label": "mitochondrion",
  "gene": "UniProtKB:Q9Y241",
  "gene_symbol": "HIGD1A",
  "gene_name": "HIG1 domain family member 1A, mitochondrial",
  "term_id": "GO:0005739"
}